{
  "gene": "UniProtKB:O14576",
  "term_label": "dynein light chain binding",
  "term_id": "GO:0045503",
  "gene_symbol": "DYNC1I1",
  "gene_name": "Cytoplasmic dynein 1 intermediate chain 1"
}